{
  "gene_name": "Glycerol kinase 3",
  "term_label": "glycerol-3-phosphate biosynthetic process",
  "gene": "UniProtKB:Q14409",
  "gene_symbol": "GK3",
  "term_id": "GO:0046167"
}